5'-flap endonuclease activity [GO:0017108] (molecular function) Definition: Catalysis of the cleavage of a 5' flap structure in DNA, but not other DNA structures; processes the 5' ends of Okazaki fragments in lagging strand DNA synthesis. Relationships: is a type of DNA endonuclease activity, producing 5'-phosphomonoesters [GO:0016888]; is a type of flap endonuclease activity [GO:0048256] Also known as: 5' flap endonuclease activity References: PMID:9778254